shoot system morphogenesis [GO:0010016] (biological process) Also known as: shoot morphogenesis Regulation: regulated by regulation of shoot system morphogenesis [GO:1900618] Relationships: is a type of anatomical structure morphogenesis [GO:0009653]; is part of shoot system development [GO:0048367] Sources: GOC:sm, ISBN:0877797099 Subtypes: GO:0010064, inflorescence morphogenesis [GO:0048281], flower morphogenesis [GO:0048439] Definition: The process in which the anatomical structures of the shoot are generated and organized. The shoot is the part of a seed plant body that is usually above ground.